{
  "gene": "UniProtKB:P04053",
  "gene_name": "DNA nucleotidylexotransferase",
  "gene_symbol": "DNTT",
  "term_id": "GO:0003912",
  "term_label": "DNA nucleotidylexotransferase activity"
}